symbiont-mediated activation of host reticulophagy [GO:0140883] (biological process) References: PMID:35239449 Relationships: is a type of symbiont-mediated activation of host autophagy [GO:0039520] Definition: A process in which a symbiont initiates, promotes, or enhances the normal execution of host reticulophagy, leading to an increase in the frequency, rate or extent of reticulophagy in the host cell. The host is defined as the larger of the organisms involved in a symbiotic interaction. Also known as: positive regulation by virus of host reticulophagy, activation of host reticulophagy by virus, induction by virus of host reticulophagy